{
  "term_label": "Unknown cellular component",
  "gene_symbol": "PRG2",
  "term_id": "UNKNOWN:0003",
  "gene": "UniProtKB:P13727",
  "gene_name": "Bone marrow proteoglycan"
}